{
  "term_id": "GO:0000423",
  "gene_name": "Sorting nexin-7",
  "gene": "UniProtKB:Q9UNH6",
  "gene_symbol": "SNX7",
  "term_label": "mitophagy"
}